{
  "gene": "UniProtKB:O94868",
  "gene_symbol": "FCHSD2",
  "term_label": "neuromuscular synaptic transmission",
  "term_id": "GO:0007274",
  "gene_name": "F-BAR and double SH3 domains protein 2"
}